positive regulation of extracellular matrix disassembly [GO:0090091] (biological process) Relationships: is a type of regulation of extracellular matrix disassembly [GO:0010715]; is a type of positive regulation of extracellular matrix organization [GO:1903055]; positively regulates extracellular matrix disassembly [GO:0022617] Sources: GOC:dph, GOC:tb Definition: Any process that increases the rate, frequency or extent of extracellular matrix disassembly. Extracellular matrix disassembly is a process that results in the breakdown of the extracellular matrix.